sialic acid:proton symporter activity [GO:0015538] (molecular function) Sources: TC:2.A.1.12.1 Relationships: is_a sialic acid transmembrane transporter activity [GO:0015136]; is_a solute:proton symporter activity [GO:0015295] Definition: Enables the transfer of a solute or solutes from one side of a membrane to the other according to the reaction: sialate(out) + H+(out) = sialate(in) + H+(in). Also known as: sialic acid:hydrogen symporter activity, sialic acid permease activity